translation factor activity, non-nucleic acid binding [GO:0045183] (molecular function) Relationships: is a type of translation factor activity [GO:0180051] Definition: A translation regulator activity that does not involve binding to nucleic acids. Sources: GOC:ai, GOC:dph, GOC:tb